{
  "term_id": "GO:0044528",
  "gene_symbol": "FASTKD3",
  "term_label": "regulation of mitochondrial mRNA stability",
  "gene_name": "FAST kinase domain-containing protein 3, mitochondrial",
  "gene": "UniProtKB:Q14CZ7"
}